{
  "term_id": "GO:0003700",
  "gene_symbol": "ZNF383",
  "gene": "UniProtKB:Q8NA42",
  "gene_name": "Zinc finger protein 383",
  "term_label": "DNA-binding transcription factor activity"
}